negative regulation of renal amino acid absorption [GO:1902753] (biological process) Definition: Any process that stops, prevents or reduces the frequency, rate or extent of renal amino acid absorption. References: PMID:1526373 Sources: GOC:TermGenie, GOC:hjd, GO_REF:0000058 Relationships: is a type of negative regulation of multicellular organismal process [GO:0051241]; is a type of regulation of renal amino acid absorption [GO:1902752]; negatively regulates renal amino acid absorption [GO:1990297] Also known as: down regulation of renal amino acid absorption, down-regulation of renal amino acid absorption, downregulation of renal amino acid absorption, inhibition of renal amino acid absorption